{
  "term_id": "UNKNOWN:0003",
  "gene": "UniProtKB:A8K0R7",
  "gene_symbol": "ZNF839",
  "gene_name": "Zinc finger protein 839",
  "term_label": "Unknown cellular component"
}